{
  "term_label": "branched-chain alpha-ketoacid dehydrogenase complex",
  "gene_symbol": "BCKDHB",
  "term_id": "GO:0160157",
  "gene_name": "2-oxoisovalerate dehydrogenase subunit beta, mitochondrial",
  "gene": "UniProtKB:P21953"
}